{
  "gene_name": "Alpha-2-HS-glycoprotein",
  "term_id": "GO:0030502",
  "term_label": "negative regulation of bone mineralization",
  "gene_symbol": "AHSG",
  "gene": "UniProtKB:P02765"
}